{
  "term_id": "GO:0017158",
  "gene_symbol": "SYT9",
  "gene": "UniProtKB:Q86SS6",
  "gene_name": "Synaptotagmin-9",
  "term_label": "regulation of calcium ion-dependent exocytosis"
}